Lid2 complex [GO:0048189] (cellular component) Definition: A protein complex involved in regulation of chromatin remodeling. In Schizosaccharomyces the complex contains Lid2, Ash2, Jmj3, Snt2, and Sdc1. Relationships: is a type of nuclear protein-containing complex [GO:0140513] References: PMID:12488447